{
  "gene_symbol": "IMP3",
  "term_id": "GO:0030515",
  "term_label": "snoRNA binding",
  "gene": "UniProtKB:Q9NV31",
  "gene_name": "U3 small nucleolar ribonucleoprotein protein IMP3"
}